{
  "gene_name": "P2Y purinoceptor 2",
  "term_label": "G protein-coupled receptor signaling pathway",
  "term_id": "GO:0007186",
  "gene": "UniProtKB:P41231",
  "gene_symbol": "P2RY2"
}